{
  "term_label": "Unknown molecular function",
  "gene_name": "T cell receptor alpha joining 33 (Fragment)",
  "gene_symbol": "TRAJ33",
  "gene": "UniProtKB:A0A075B6W3",
  "term_id": "UNKNOWN:0001"
}